U6atac snRNA binding [GO:0030624] (molecular function) Definition: Binding to a U6atac small nuclear RNA (U6atac snRNA). Sources: GOC:jl Relationships: is a type of snRNA binding [GO:0017069]